regulation of kinase activity [GO:0043549] (biological process) Subtypes: negative regulation of kinase activity [GO:0033673], GO:0033674, regulation of lipid kinase activity [GO:0043550], regulation of protein kinase activity [GO:0045859] Sources: GOC:bf Relationships: is a type of regulation of phosphorylation [GO:0042325]; is a type of regulation of transferase activity [GO:0051338]; RO_0002211 GO:0016301 Definition: Any process that modulates the frequency, rate or extent of kinase activity, the catalysis of the transfer of a phosphate group, usually from ATP, to a substrate molecule.